3-hydroxybutyryl-CoA dehydrogenase activity [GO:0008691] (molecular function) Sources: EC:1.1.1.157 Also known as: (S)-3-hydroxybutanoyl-CoA:NADP+ oxidoreductase activity, BHBD activity, L(+)-3-hydroxybutyryl-CoA dehydrogenase activity, L-(+)-3-hydroxybutyryl-CoA dehydrogenase activity, beta-hydroxybutyryl coenzyme A dehydrogenase activity, beta-hydroxybutyryl-CoA dehydrogenase activity, dehydrogenase, L-3-hydroxybutyryl coenzyme A (nicotinamide adenine dinucleotide phosphate) Relationships: is a type of oxidoreductase activity, acting on the CH-OH group of donors, NAD or NADP as acceptor [GO:0016616] Definition: Catalysis of the reaction: (S)-3-hydroxybutanoyl-CoA + NADP+ = 3-acetoacetyl-CoA + NADPH + H+.